{
  "gene": "UniProtKB:A0A8V8TNB9",
  "term_id": "UNKNOWN:0002",
  "gene_name": "Uncharacterized protein",
  "gene_symbol": "A0A8V8TNB9",
  "term_label": "Unknown biological process"
}